{
  "gene": "UniProtKB:A6NI86",
  "gene_symbol": "GOLGA6L10",
  "gene_name": "Golgin subfamily A member 6-like protein 10",
  "term_label": "Unknown cellular component",
  "term_id": "UNKNOWN:0003"
}